{
  "gene_name": "Tigger transposable element-derived protein 5",
  "term_label": "Unknown biological process",
  "gene_symbol": "TIGD5",
  "term_id": "UNKNOWN:0002",
  "gene": "UniProtKB:Q53EQ6"
}